{
  "gene_symbol": "PPP1R11",
  "term_id": "GO:0004865",
  "gene_name": "E3 ubiquitin-protein ligase PPP1R11",
  "term_label": "protein serine/threonine phosphatase inhibitor activity",
  "gene": "UniProtKB:O60927"
}